{
  "gene_symbol": "NEDD8",
  "term_id": "GO:0045116",
  "term_label": "protein neddylation",
  "gene": "UniProtKB:Q15843",
  "gene_name": "NEDD8"
}